{
  "gene_name": "CHRNA7-FAM7A fusion protein",
  "gene": "UniProtKB:Q494W8",
  "term_id": "GO:0034220",
  "gene_symbol": "CHRFAM7A",
  "term_label": "monoatomic ion transmembrane transport"
}